{
  "term_label": "guanyl-nucleotide exchange factor activity",
  "gene": "UniProtKB:Q9NQG7",
  "gene_name": "BLOC-3 complex member HPS4",
  "term_id": "GO:0005085",
  "gene_symbol": "HPS4"
}